{
  "gene_symbol": "STX6",
  "gene_name": "Syntaxin-6",
  "gene": "UniProtKB:O43752",
  "term_label": "vesicle docking",
  "term_id": "GO:0048278"
}